compound eye cone cell fate commitment [GO:0042676] (biological process) Relationships: is a type of GO:0045165; BFO_0000050 compound eye cone cell differentiation [GO:0042675] Sources: GOC:mtg_sensu Definition: The process in which the cone cells of the compound eye, the lens-secreting cells in the ommatidia, adopt pathways of differentiation that lead to the establishment of their distinct cell type.